{
  "term_id": "UNKNOWN:0001",
  "term_label": "Unknown molecular function",
  "gene": "UniProtKB:Q9H1P6",
  "gene_symbol": "C20orf85",
  "gene_name": "Uncharacterized protein C20orf85"
}